{
  "term_label": "actin binding",
  "gene_symbol": "EMD",
  "gene": "UniProtKB:P50402",
  "gene_name": "Emerin",
  "term_id": "GO:0003779"
}